{
  "gene_name": "Transcription factor HES-1",
  "gene": "UniProtKB:Q14469",
  "term_id": "GO:0070888",
  "gene_symbol": "HES1",
  "term_label": "E-box binding"
}